{
  "gene": "UniProtKB:A0A2R8YFL7",
  "term_label": "Unknown biological process",
  "term_id": "UNKNOWN:0002",
  "gene_name": "Oocyte-secreted protein 4A",
  "gene_symbol": "OOSP4A"
}